CatSper complex [GO:0036128] (cellular component) References: PMID:17478420, PMID:21224844, PMID:22354039 Sources: GOC:sp Definition: A sperm-specific voltage-gated calcium channel that controls the intracellular calcium ion concentration and, thereby, the swimming behavior of sperm. Consists of a heteromeric tetramer surrounding a calcium ion- selective pore. May also contain additional auxiliary subunits. Relationships: is a type of voltage-gated calcium channel complex [GO:0005891] Also known as: CATSPER channel, CatSper channel complex